neuregulin binding [GO:0038132] (molecular function) Sources: GOC:bf, GOC:signaling Relationships: is a type of growth factor binding [GO:0019838] Definition: Binding to a neuregulin, a member of the EGF family of growth factors.